{
  "gene_name": "Centromere protein W",
  "term_label": "kinetochore assembly",
  "gene": "UniProtKB:Q5EE01",
  "term_id": "GO:0051382",
  "gene_symbol": "CENPW"
}